{
  "term_id": "GO:0022625",
  "gene": "UniProtKB:P62424",
  "gene_symbol": "RPL7A",
  "gene_name": "Large ribosomal subunit protein eL8",
  "term_label": "cytosolic large ribosomal subunit"
}